{
  "gene_name": "Splicing factor, arginine_serine-rich 19",
  "term_label": "Unknown cellular component",
  "term_id": "UNKNOWN:0003",
  "gene_symbol": "SCAF1",
  "gene": "UniProtKB:Q9H7N4"
}